tRNA pseudouridine synthase activity [GO:0106029] (molecular function) References: PMID:11095668 Relationships: is a type of GO:0009982; is a type of GO:0140101 Also known as: tRNA-pseudouridine synthase activity, tRNA-uridine isomerase activity, tRNA-uridine uracilmutase activity, transfer RNA pseudouridine synthetase activity, transfer ribonucleate pseudouridine synthetase activity Subtypes: tRNA pseudouridine(38-40) synthase activity [GO:0160147], tRNA pseudouridine(55) synthase activity [GO:0160148], GO:0160149, tRNA pseudouridine(13) synthase activity [GO:0160150], tRNA pseudouridine(32) synthase activity [GO:0160151], GO:0160152, GO:0160153, tRNA pseudouridine(38/39) synthase activity [GO:0160154] Definition: Catalysis of the reaction: tRNA uridine = tRNA pseudouridine. Conversion of uridine in a tRNA molecule to pseudouridine by rotation of the C1'-N-1 glycosidic bond of uridine in RNA to a C1'-C5.